{
  "term_label": "condensed chromosome, centromeric region",
  "gene_symbol": "SYCP2L",
  "term_id": "GO:0000779",
  "gene_name": "Synaptonemal complex protein 2-like",
  "gene": "UniProtKB:Q5T4T6"
}